alignment of 3' and 5' splice sites of mRNA [GO:0034403] (biological process) Definition: Recognition of both the 5' and 3'-splice sites and positioning them in the correct alignment with respect to each other so that the second catalytic step of nuclear mRNA splicing can occur. References: PMID:9430647 Sources: GOC:krc Also known as: alignment of 3' and 5' splice sites of nuclear mRNA Relationships: is a type of mRNA 3'-splice site recognition [GO:0000389]; is a type of mRNA 5'-splice site recognition [GO:0000395]; is part of GO:0000350